{
  "term_label": "poly(A) binding",
  "gene_name": "RNA-binding motif, single-stranded-interacting protein 2",
  "term_id": "GO:0008143",
  "gene_symbol": "RBMS2",
  "gene": "UniProtKB:Q15434"
}